{
  "gene_name": "Heat shock cognate 71 kDa protein",
  "gene": "UniProtKB:P11142",
  "gene_symbol": "HSPA8",
  "term_label": "ATP hydrolysis activity",
  "term_id": "GO:0016887"
}